{
  "term_label": "DNA-binding transcription activator activity, RNA polymerase II-specific",
  "gene_name": "Zinc finger protein 784",
  "term_id": "GO:0001228",
  "gene": "UniProtKB:Q8NCA9",
  "gene_symbol": "ZNF784"
}